{
  "term_label": "Unknown molecular function",
  "gene": "UniProtKB:P48651",
  "gene_name": "Phosphatidylserine synthase 1",
  "gene_symbol": "PTDSS1",
  "term_id": "UNKNOWN:0001"
}